{
  "term_label": "actin filament binding",
  "gene": "UniProtKB:Q9Y2K3",
  "gene_symbol": "MYH15",
  "gene_name": "Myosin-15",
  "term_id": "GO:0051015"
}